multimeric ribonuclease P complex [GO:0030681] (cellular component) Relationships: is a type of ribonuclease P complex [GO:0030677] Also known as: multimeric RNase P complex Definition: A ribonuclease P complex that generally contains a single RNA molecule and several protein molecules. Examples of this complex are found in Archaeal species. References: PMID:11142368, PMID:12045094 Sources: GOC:mah Subtypes: nucleolar ribonuclease P complex [GO:0005655], cyanelle ribonuclease P complex [GO:0030679]